{
  "term_id": "UNKNOWN:0001",
  "gene_name": "Probable inactive ribonuclease-like protein 13",
  "term_label": "Unknown molecular function",
  "gene": "UniProtKB:Q5GAN3",
  "gene_symbol": "RNASE13"
}